production of molecular mediator of immune response [GO:0002440] (biological process) Also known as: production of cellular mediator of immune response Regulation: regulated by regulation of production of molecular mediator of immune response [GO:0002700]; negatively regulated by negative regulation of production of molecular mediator of immune response [GO:0002701]; positively regulated by positive regulation of production of molecular mediator of immune response [GO:0002702] Definition: The synthesis or release of any molecular mediator of the immune response, resulting in an increase in its intracellular or extracellular levels. Note: Note that this term is in the subset of terms that should not be used for direct gene product annotation. Instead, select one of the 'regulation' children terms. Relationships: is a type of immune system process [GO:0002376]; is a type of gene expression [GO:0010467] Sources: GOC:add, GO_REF:0000022, ISBN:0781735149 Subtypes: cytokine production involved in immune response [GO:0002367], GO:0002377, antimicrobial peptide production [GO:0002775], GO:0035746, GO:0035944, GO:0036262, granzyme B production [GO:0071613]